{
  "term_id": "GO:0000398",
  "gene_name": "Heterogeneous nuclear ribonucleoprotein A1",
  "gene_symbol": "HNRNPA1",
  "term_label": "mRNA splicing, via spliceosome",
  "gene": "UniProtKB:P09651"
}